{
  "term_id": "UNKNOWN:0002",
  "term_label": "Unknown biological process",
  "gene_name": "Arylacetamide deacetylase-like 3",
  "gene": "UniProtKB:Q5VUY0",
  "gene_symbol": "AADACL3"
}